{
  "term_id": "GO:0005643",
  "term_label": "nuclear pore",
  "gene_name": "Nuclear pore complex protein Nup93",
  "gene": "UniProtKB:Q8N1F7",
  "gene_symbol": "NUP93"
}